{
  "term_id": "GO:0004053",
  "gene_name": "Arginase-2, mitochondrial",
  "gene": "UniProtKB:P78540",
  "term_label": "arginase activity",
  "gene_symbol": "ARG2"
}